{
  "gene": "UniProtKB:Q9H9C1",
  "term_id": "UNKNOWN:0001",
  "term_label": "Unknown molecular function",
  "gene_name": "Spermatogenesis-defective protein 39 homolog",
  "gene_symbol": "VIPAS39"
}